{
  "gene_symbol": "COL10A1",
  "gene_name": "Collagen alpha-1(X) chain",
  "term_label": "extracellular matrix",
  "term_id": "GO:0031012",
  "gene": "UniProtKB:Q03692"
}